{
  "gene_name": "Lactoylglutathione lyase",
  "gene": "UniProtKB:Q04760",
  "term_label": "Unknown biological process",
  "term_id": "UNKNOWN:0002",
  "gene_symbol": "GLO1"
}